{
  "gene_name": "Vitamin K epoxide reductase complex subunit 1",
  "term_id": "UNKNOWN:0003",
  "gene_symbol": "VKORC1",
  "term_label": "Unknown cellular component",
  "gene": "UniProtKB:Q9BQB6"
}